{
  "term_id": "UNKNOWN:0001",
  "gene_name": "Leucine-rich repeat-containing protein 53",
  "term_label": "Unknown molecular function",
  "gene": "UniProtKB:A6NM62",
  "gene_symbol": "LRRC53"
}